{
  "term_label": "heterochromatin formation",
  "gene_symbol": "CBX1",
  "gene": "UniProtKB:P83916",
  "gene_name": "Chromobox protein homolog 1",
  "term_id": "GO:0031507"
}